plasma membrane of growing cell tip [GO:1902929] (cellular component) Definition: Any plasma membrane part that is part of a growing cell tip. References: PMID:17085965 Sources: GOC:TermGenie, GO_REF:0000064 Also known as: growing cell tip plasma membrane part, plasma membrane part of growing cell end, plasma membrane part of growing cell tip Relationships: is a type of GO:0031520; is part of growing cell tip [GO:0035838]